{
  "gene_symbol": "USP24",
  "gene": "UniProtKB:Q9UPU5",
  "term_id": "GO:0031647",
  "gene_name": "Ubiquitin carboxyl-terminal hydrolase 24",
  "term_label": "regulation of protein stability"
}